{
  "gene_name": "Splicing factor 3B subunit 5",
  "gene_symbol": "SF3B5",
  "term_label": "U2 snRNP",
  "gene": "UniProtKB:Q9BWJ5",
  "term_id": "GO:0005686"
}